positive regulation of emericellamide biosynthetic process [GO:1900660] (BP) Subtypes: GO:1900663 Relationships: is a type of GO:0034250; is a type of GO:0046889; is a type of positive regulation of small molecule metabolic process [GO:0062013]; is a type of positive regulation of secondary metabolite biosynthetic process [GO:1900378]; is a type of GO:1900658; positively regulates emericellamide biosynthetic process [GO:1900557] Sources: GOC:TermGenie, GOC:di Definition: Any process that activates or increases the frequency, rate or extent of emericellamide biosynthetic process. Also known as: activation of emericellamide anabolism, activation of emericellamide biosynthesis, activation of emericellamide formation, activation of emericellamide synthesis, positive regulation of emericellamide anabolism, positive regulation of emericellamide biosynthesis, positive regulation of emericellamide formation, positive regulation of emericellamide synthesis, up regulation of emericellamide anabolism, up regulation of emericellamide biosynthesis, up regulation of emericellamide biosynthetic process, up regulation of emericellamide formation, up regulation of emericellamide synthesis, up-regulation of emericellamide anabolism, up-regulation of emericellamide biosynthesis, up-regulation of emericellamide biosynthetic process, up-regulation of emericellamide formation, up-regulation of emericellamide synthesis, upregulation of emericellamide anabolism, upregulation of emericellamide biosynthesis, upregulation of emericellamide biosynthetic process, upregulation of emericellamide formation, upregulation of emericellamide synthesis, activation of emericellamide biosynthetic process